negative regulation of JUN kinase activity [GO:0043508] (biological process) Relationships: is a type of negative regulation of MAP kinase activity [GO:0043407]; is a type of regulation of JUN kinase activity [GO:0043506]; is_a GO:0046329; negatively regulates GO:0004705 Definition: Any process that stops, prevents, or reduces the frequency, rate or extent of JUN kinase activity. Sources: GOC:jl Also known as: down regulation of JNK activity, down-regulation of JNK activity, downregulation of JNK activity, negative regulation of JUNK activity, inhibition of JNK activity